{
  "gene_name": "cAMP-dependent protein kinase inhibitor gamma",
  "term_id": "GO:0004862",
  "term_label": "cAMP-dependent protein kinase inhibitor activity",
  "gene_symbol": "PKIG",
  "gene": "UniProtKB:Q9Y2B9"
}